{
  "gene_name": "Serpin B10",
  "term_label": "serine-type endopeptidase inhibitor activity",
  "term_id": "GO:0004867",
  "gene_symbol": "SERPINB10",
  "gene": "UniProtKB:P48595"
}